phosphoenolpyruvate mutase activity [GO:0050188] (molecular function) Relationships: is a type of intramolecular phosphotransferase activity [GO:0016868] Definition: Catalysis of the reaction: phosphoenolpyruvate = 3-phosphonopyruvate. Sources: EC:5.4.2.9, RHEA:17013 Also known as: PEP mutase activity, PEP phosphomutase activity, PEPPM, phosphoenolpyruvate 2,3-phosphonomutase activity, phosphoenolpyruvate phosphomutase activity, phosphoenolpyruvate-phosphonopyruvate phosphomutase activity